{
  "gene": "UniProtKB:Q9NP08",
  "gene_symbol": "HMX1",
  "gene_name": "Homeobox protein HMX1",
  "term_label": "DNA-binding transcription factor activity, RNA polymerase II-specific",
  "term_id": "GO:0000981"
}